corticospinal neuron axon guidance through the basilar pons [GO:0021970] (biological process) Definition: The process in which the migration of an axon growth cone of a pyramidal cell that is part of the corticospinal tract is directed after exiting the cerebral peduncle through the basilar pons in response to a combination of attractive and repulsive cues. Relationships: is a type of GO:0007411; BFO_0000050 GO:0021966 Also known as: corticospinal neuron axon pathfinding through the basilar pons References: PMID:9878731 Sources: GOC:cls, GOC:dgh, GOC:dph, GOC:jid, GO_REF:0000021